{
  "gene_symbol": "PFN1",
  "term_id": "GO:0003779",
  "term_label": "actin binding",
  "gene": "UniProtKB:P07737",
  "gene_name": "Profilin-1"
}